mesonephric renal vesicle morphogenesis [GO:0061243] (biological process) Relationships: is_a renal vesicle morphogenesis [GO:0072077]; is part of mesonephric nephron morphogenesis [GO:0061228] Definition: The process in which the anatomical structures of the mesonephric renal vesicle are generated and organized. The renal vesicle is the primordial structure of the mesonephric nephron epithelium, and is formed by the condensation of mesenchymal cells. Sources: GOC:mtg_kidney_jan10